gliogenesis [GO:0042063] (biological process) Relationships: is a type of neurogenesis [GO:0022008] Definition: The process that results in the generation of glial cells. This includes the production of glial progenitors and their differentiation into mature glia. Also known as: glial cell generation Sources: GOC:dgh, GOC:jid Regulation: regulated by regulation of gliogenesis [GO:0014013]; negatively regulated by negative regulation of gliogenesis [GO:0014014]; positively regulated by positive regulation of gliogenesis [GO:0014015]